{
  "term_label": "G protein-coupled receptor signaling pathway",
  "gene_symbol": "OR5D14",
  "gene_name": "Olfactory receptor 5D14",
  "gene": "UniProtKB:Q8NGL3",
  "term_id": "GO:0007186"
}